negative regulation of cell motility involved in cerebral cortex radial glia guided migration [GO:0021822] (biological process) Relationships: is a type of negative regulation of glial cell migration [GO:1903976]; is part of layer formation in cerebral cortex [GO:0021819]; negatively regulates GO:0021814 Definition: The intracellular signaling pathway that results in the cessation of cell movement involved in lamination of the cerebral cortex. References: PMID:12626695 Sources: GOC:cls, GOC:dgh, GOC:dph, GOC:jid, GOC:tb Also known as: down regulation of cell locomotion involved in cerebral cortex glial-mediated radial cell migration, down-regulation of cell locomotion involved in cerebral cortex glial-mediated radial cell migration, downregulation of cell locomotion involved in cerebral cortex glial-mediated radial cell migration, negative regulation of cell locomotion involved in cerebral cortex glial-mediated radial migration, inhibition of cell locomotion involved in cerebral cortex glial-mediated radial cell migration, negative regulation of cell locomotion involved in cerebral cortex radial glia guided migration